{
  "term_label": "positive regulation of neuron apoptotic process",
  "term_id": "GO:0043525",
  "gene_name": "Glycogen synthase kinase-3 beta",
  "gene_symbol": "GSK3B",
  "gene": "UniProtKB:P49841"
}